{
  "term_id": "GO:0005737",
  "gene_name": "Suppressor of fused homolog",
  "gene": "UniProtKB:Q9UMX1",
  "gene_symbol": "SUFU",
  "term_label": "cytoplasm"
}